{
  "term_id": "GO:0005315",
  "gene_symbol": "ANKH",
  "gene_name": "Progressive ankylosis protein homolog",
  "term_label": "phosphate transmembrane transporter activity",
  "gene": "UniProtKB:Q9HCJ1"
}